{
  "term_id": "GO:0005634",
  "gene": "UniProtKB:O15062",
  "term_label": "nucleus",
  "gene_symbol": "ZBTB5",
  "gene_name": "Zinc finger and BTB domain-containing protein 5"
}